{
  "gene_name": "Rho GTPase-activating protein 5",
  "gene_symbol": "ARHGAP5",
  "term_id": "GO:0005829",
  "gene": "UniProtKB:Q13017",
  "term_label": "cytosol"
}